{
  "term_id": "GO:0005886",
  "gene_symbol": "LIMA1",
  "gene_name": "LIM domain and actin-binding protein 1",
  "gene": "UniProtKB:Q9UHB6",
  "term_label": "plasma membrane"
}